{
  "term_label": "Unknown molecular function",
  "gene": "UniProtKB:Q14134",
  "term_id": "UNKNOWN:0001",
  "gene_name": "Tripartite motif-containing protein 29",
  "gene_symbol": "TRIM29"
}